cell fate specification involved in pattern specification [GO:0060573] (biological process) Subtypes: GO:0021521, notum cell fate specification [GO:0035310], wing cell fate specification [GO:0035311], limb basal epidermal cell fate specification [GO:0060892], GO:0060893, limb spinous cell fate specification [GO:0060894] Definition: The process involved in the specification of the identity of a cell in a field of cells that is being instructed as to how to differentiate. Once specification has taken place, that cell will be committed to differentiate down a specific pathway if left in its normal environment. Relationships: is a type of GO:0001708; is part of cell fate commitment involved in pattern specification [GO:0060581] Sources: GOC:dph, GOC:tb